cutin-based cuticle development [GO:0160062] (biological process) References: PMID:23893170 Relationships: is a type of anatomical structure development [GO:0048856] Definition: The process whose specific outcome is the progression of the cutin-based cuticle over time, from its formation to the mature structure. Cutin-based cuticle is an extracellular structure composed of a covalently linked macromolecular scaffold of cutin and a variety of organic solvent-soluble lipids that are collectively termed waxes. Such structures are found on the external face of polysaccharide cell walls in land plants.